{
  "gene_name": "Kinesin-like protein KIFC1",
  "gene": "UniProtKB:Q9BW19",
  "term_id": "GO:0007018",
  "gene_symbol": "KIFC1",
  "term_label": "microtubule-based movement"
}